{
  "term_id": "GO:0008270",
  "gene_name": "Lipopolysaccharide-induced tumor necrosis factor-alpha factor",
  "gene_symbol": "LITAF",
  "term_label": "zinc ion binding",
  "gene": "UniProtKB:Q99732"
}